negative regulation of activation-induced cell death of T cells [GO:0070236] (biological process) Sources: GOC:add, ISBN:0781765196 Also known as: negative regulation of AICD, negative regulation of activated T cell apoptosis, negative regulation of antigen-driven apoptosis, down regulation of activation-induced cell death of T cells, down-regulation of activation-induced cell death of T cells, downregulation of activation-induced cell death of T cells, negative regulation of activation-induced cell death of T lymphocytes, negative regulation of activation-induced cell death of T-cells, negative regulation of activation-induced cell death of T-lymphocytes, inhibition of activation-induced cell death of T cells Definition: Any process that stops, prevents, or reduces the frequency, rate or extent of activation-induced cell death of T cells. Relationships: is a type of negative regulation of immune system process [GO:0002683]; is a type of negative regulation of T cell apoptotic process [GO:0070233]; is a type of regulation of activation-induced cell death of T cells [GO:0070235]; negatively regulates activation-induced cell death of T cells [GO:0006924]